{
  "gene_symbol": "SLC25A5",
  "gene_name": "ADP_ATP translocase 2",
  "term_label": "regulation of mitochondrial membrane permeability",
  "gene": "UniProtKB:P05141",
  "term_id": "GO:0046902"
}